cytoplasmic microtubule minus-end [GO:0062194] (cellular component) Definition: A microtubule minus end that is part of a cytoplasmic microtubule. References: PMID:18061564 Relationships: is a type of microtubule minus-end [GO:0036449]; BFO_0000050 GO:0005881